fatty acid transmembrane transport [GO:1902001] (biological process) Relationships: is a type of fatty acid transport [GO:0015908]; is a type of GO:1905039 References: PMID:9395310 Sources: GOC:TermGenie, GOC:rb Subtypes: carnitine shuttle [GO:0006853], long-chain fatty acid import into peroxisome [GO:0015910], long-chain fatty acid import across plasma membrane [GO:0015911], GO:0015913 Definition: The process in which a fatty acid is transported across a membrane.